{
  "term_id": "UNKNOWN:0003",
  "gene": "UniProtKB:Q9BTT4",
  "gene_symbol": "MED10",
  "gene_name": "Mediator of RNA polymerase II transcription subunit 10",
  "term_label": "Unknown cellular component"
}